{
  "gene_symbol": "VCL",
  "gene": "UniProtKB:P18206",
  "gene_name": "Vinculin",
  "term_label": "cell-cell contact zone",
  "term_id": "GO:0044291"
}